{
  "term_id": "GO:0005737",
  "gene_symbol": "CDC123",
  "gene_name": "Cell division cycle protein 123 homolog",
  "gene": "UniProtKB:O75794",
  "term_label": "cytoplasm"
}